{
  "gene_name": "Mediator of RNA polymerase II transcription subunit 6",
  "gene": "UniProtKB:O75586",
  "term_label": "transcription coactivator activity",
  "term_id": "GO:0003713",
  "gene_symbol": "MED6"
}